Gram-positive-bacterium-type cell wall [GO:0009275] (cellular component) Definition: A layer of peptidoglycan found outside of the cytoplasmic membrane. The peptidoglycan is relatively thick (20-80nm) and retains the primary stain of the Gram procedure, thus cells appear blue after Gram stain. The cell walls often contain teichoic acids (acidic anionic polysaccharides) bound to the peptidoglycan. Examples of this component are found in Gram-positive bacteria. Sources: GOC:mlg, ISBN:0815108893 Relationships: is a type of peptidoglycan-based cell wall [GO:0009274] Also known as: 20-80nm peptidoglycan-based cell wall, cell wall of Gram-positive Bacteria